{
  "term_id": "GO:0051965",
  "gene": "UniProtKB:O94991",
  "gene_name": "SLIT and NTRK-like protein 5",
  "gene_symbol": "SLITRK5",
  "term_label": "positive regulation of synapse assembly"
}